{
  "term_id": "GO:0005634",
  "gene": "UniProtKB:Q9ULD4",
  "term_label": "nucleus",
  "gene_symbol": "BRPF3",
  "gene_name": "Bromodomain and PHD finger-containing protein 3"
}